{
  "gene_name": "Myosin regulatory light chain 2, ventricular_cardiac muscle isoform",
  "gene_symbol": "MYL2",
  "term_label": "calcium ion binding",
  "gene": "UniProtKB:P10916",
  "term_id": "GO:0005509"
}